{
  "term_label": "transcription coregulator activity",
  "gene_name": "Zinc finger protein ZXDC",
  "gene_symbol": "ZXDC",
  "term_id": "GO:0003712",
  "gene": "UniProtKB:Q2QGD7"
}